extracellular amino acid transport [GO:0006860] (biological process) Sources: GOC:ai Relationships: is a type of extracellular transport [GO:0006858]; is a type of GO:0006865 Definition: The directed extracellular movement of amino acids.